{
  "term_id": "GO:0006888",
  "gene_symbol": "SEC22A",
  "gene": "UniProtKB:Q96IW7",
  "gene_name": "Vesicle-trafficking protein SEC22a",
  "term_label": "endoplasmic reticulum to Golgi vesicle-mediated transport"
}